{
  "term_id": "UNKNOWN:0003",
  "gene": "UniProtKB:Q9UIG4",
  "gene_name": "Psoriasis susceptibility 1 candidate gene 2 protein",
  "gene_symbol": "PSORS1C2",
  "term_label": "Unknown cellular component"
}